{
  "gene": "UniProtKB:P15151",
  "term_label": "natural killer cell mediated cytotoxicity",
  "gene_symbol": "PVR",
  "term_id": "GO:0042267",
  "gene_name": "Poliovirus receptor"
}